{
  "gene_name": "Interferon alpha-7",
  "term_label": "extracellular space",
  "gene_symbol": "IFNA7",
  "term_id": "GO:0005615",
  "gene": "UniProtKB:P01567"
}